peptidoglycan beta-N-acetylmuramidase activity [GO:0033922] (molecular function) Definition: Catalysis of the hydrolysis of terminal, non-reducing N-acetylmuramic residues. Sources: EC:3.2.1.92 Also known as: beta-2-acetamido-3-O-(D-1-carboxyethyl)-2-deoxy-D-glucoside acetamidodeoxyglucohydrolase activity, exo-beta-N-acetylmuramidase activity, exo-beta-acetylmuramidase activity, peptidoglycan beta-N-acetylmuramoylexohydrolase activity Relationships: is a type of hydrolase activity, hydrolyzing O-glycosyl compounds [GO:0004553]